long tract gene conversion [GO:0035824] (biological process) Definition: A gene conversion process in which a segment of more than 1000 base pairs is transferred from the donor to the acceptor. Relationships: is a type of gene conversion [GO:0035822] References: PMID:16954385 Sources: GOC:mah